negative regulation of sensory perception of bitter taste [GO:1904661] (biological process) Relationships: is a type of negative regulation of nervous system process [GO:0031645]; is a type of GO:1904660; negatively regulates sensory perception of bitter taste [GO:0050913] References: PMID:1716172 Sources: GOC:TermGenie, GOC:mr, GO_REF:0000058 Definition: Any process that stops, prevents or reduces the frequency, rate or extent of sensory perception of bitter taste. Also known as: down regulation of bitter taste perception, down regulation of sensory perception of bitter taste, down-regulation of bitter taste perception, down-regulation of sensory perception of bitter taste, downregulation of bitter taste perception, downregulation of sensory perception of bitter taste, negative regulation of bitter taste perception, inhibition of bitter taste perception, inhibition of sensory perception of bitter taste